{
  "term_label": "immune response",
  "gene": "UniProtKB:A0A0B4J2D9",
  "gene_name": "Immunoglobulin kappa variable 1D-13",
  "gene_symbol": "IGKV1D-13",
  "term_id": "GO:0006955"
}